{
  "gene_name": "N-alpha-acetyltransferase 38, NatC auxiliary subunit",
  "gene_symbol": "NAA38",
  "gene": "UniProtKB:Q9BRA0",
  "term_label": "Unknown molecular function",
  "term_id": "UNKNOWN:0001"
}